{
  "gene_symbol": "TENM2",
  "gene": "UniProtKB:Q9NT68",
  "term_id": "GO:0042803",
  "gene_name": "Teneurin-2",
  "term_label": "protein homodimerization activity"
}